{
  "gene_name": "Sorting nexin-33",
  "term_label": "cytoplasmic vesicle",
  "gene": "UniProtKB:Q8WV41",
  "gene_symbol": "SNX33",
  "term_id": "GO:0031410"
}